{
  "gene_symbol": "ESS2",
  "term_label": "catalytic step 2 spliceosome",
  "gene": "UniProtKB:Q96DF8",
  "term_id": "GO:0071013",
  "gene_name": "Splicing factor ESS-2 homolog"
}